{
  "gene_name": "Protein-lysine 6-oxidase",
  "gene_symbol": "LOX",
  "term_id": "GO:0004720",
  "gene": "UniProtKB:P28300",
  "term_label": "protein-lysine 6-oxidase activity"
}